{
  "term_label": "cell surface",
  "term_id": "GO:0009986",
  "gene": "UniProtKB:P16671",
  "gene_symbol": "CD36",
  "gene_name": "Platelet glycoprotein 4"
}